{
  "term_id": "UNKNOWN:0003",
  "gene_name": "Platelet-activating factor acetylhydrolase 2, cytoplasmic",
  "term_label": "Unknown cellular component",
  "gene": "UniProtKB:Q99487",
  "gene_symbol": "PAFAH2"
}